{
  "gene_symbol": "HLA-DRB1",
  "term_id": "GO:0042613",
  "gene_name": "HLA class II histocompatibility antigen, DRB1 beta chain",
  "gene": "UniProtKB:P01911",
  "term_label": "MHC class II protein complex"
}